{
  "term_id": "GO:0005739",
  "gene_name": "L-lactate dehydrogenase A chain",
  "gene": "UniProtKB:P00338",
  "term_label": "mitochondrion",
  "gene_symbol": "LDHA"
}